{
  "term_id": "UNKNOWN:0001",
  "gene_symbol": "METTL8",
  "term_label": "Unknown molecular function",
  "gene": "UniProtKB:Q9H825",
  "gene_name": "tRNA N(3)-methylcytidine methyltransferase METTL8, mitochondrial"
}